proton-transporting ATP synthase complex assembly [GO:0043461] (biological process) Definition: The aggregation, arrangement and bonding together of a proton-transporting ATP synthase (also known as F-type ATPase), a two-sector ATPase found in the inner membrane of mitochondria and chloroplasts, and in bacterial plasma membranes. Relationships: is a type of GO:0070071 Also known as: F-type ATPase complex assembly Subtypes: GO:0033614, mitochondrial proton-transporting ATP synthase complex assembly [GO:0033615], plasma membrane proton-transporting ATP synthase complex assembly [GO:0033616] References: PMID:29514954 Sources: GOC:jl, GOC:mah